cerebellar cortex development [GO:0021695] (biological process) Relationships: is a type of anatomical structure development [GO:0048856]; is part of cerebellum development [GO:0021549] Sources: GOC:cls, GOC:dgh, GOC:dph, GOC:jid, GO_REF:0000021 Definition: The process whose specific outcome is the progression of the cerebellar cortex over time, from its formation to the mature structure. The cerebellar cortex is a thin mantle of gray matter that covers the surface of each cerebral hemisphere. It has a characteristic morphology with convolutions (gyri) and crevices (sulci) that have specific functions. Six layers of nerve cells and the nerve pathways that connect them comprise the cerebellar cortex. Together, these regions are responsible for the processes of conscious thought, perception, emotion and memory as well as advanced motor function.